positive regulation of steroid metabolic process [GO:0045940] (biological process) Also known as: positive regulation of steroid metabolism, up regulation of steroid metabolic process, up-regulation of steroid metabolic process, upregulation of steroid metabolic process, activation of steroid metabolic process, stimulation of steroid metabolic process Relationships: is a type of regulation of steroid metabolic process [GO:0019218]; is a type of positive regulation of lipid metabolic process [GO:0045834]; positively regulates steroid metabolic process [GO:0008202] Definition: Any process that activates or increases the frequency, rate or extent of the chemical reactions and pathways involving steroids. Sources: GOC:go_curators Subtypes: positive regulation of steroid biosynthetic process [GO:0010893], positive regulation of glucocorticoid catabolic process [GO:0031951], positive regulation of cholesterol metabolic process [GO:0090205]